{
  "term_id": "GO:0016477",
  "term_label": "cell migration",
  "gene_symbol": "CDH18",
  "gene": "UniProtKB:Q13634",
  "gene_name": "Cadherin-18"
}